{
  "term_id": "GO:0005634",
  "gene_name": "Cytosolic carboxypeptidase 1",
  "gene_symbol": "AGTPBP1",
  "gene": "UniProtKB:Q9UPW5",
  "term_label": "nucleus"
}